secondary heart field specification [GO:0003139] (biological process) Relationships: is a type of GO:0003128 References: PMID:17276708 Sources: GOC:mtg_heart, GOC:rl Definition: The process that results in the delineation of a specific region of the lateral mesoderm into the area which will form the majority of the mesodermal component of the right ventricle, arterial pole (outflow tract) and venous pole (inflow tract). Also known as: SHF specification, second heart field specification, anterior heart field specification